{
  "term_id": "UNKNOWN:0003",
  "gene_symbol": "ZNF662",
  "term_label": "Unknown cellular component",
  "gene": "UniProtKB:Q6ZS27",
  "gene_name": "Zinc finger protein 662"
}